phagocytic vesicle membrane [GO:0030670] (CC) Subtypes: GO:0030671, early phagosome membrane [GO:0036186], phagolysosome membrane [GO:0061474] Sources: GOC:mah Definition: The lipid bilayer surrounding a phagocytic vesicle. Also known as: phagosome membrane Relationships: is a type of endocytic vesicle membrane [GO:0030666]; is part of phagocytic vesicle [GO:0045335]